{
  "term_label": "wide pore channel activity",
  "gene_name": "Pannexin-2",
  "gene": "UniProtKB:Q96RD6",
  "term_id": "GO:0022829",
  "gene_symbol": "PANX2"
}